heme B catabolic process [GO:1900548] (biological process) Also known as: heme B breakdown, heme B catabolism, heme B degradation, protoheme catabolic process, protoheme degradation Definition: The chemical reactions and pathways resulting in the breakdown of heme b, a Fe(II) porphyrin complex readily isolated from the hemoglobin of beef blood, but also found in other proteins including other hemoglobins, myoglobins, cytochromes P-450, catalases, peroxidases as well as b type cytochromes. Relationships: is a type of heme catabolic process [GO:0042167] References: PMID:28352909 Sources: GOC:TermGenie, GOC:yaf